{
  "gene_name": "C-X-C chemokine receptor type 3",
  "term_id": "GO:0060326",
  "gene_symbol": "CXCR3",
  "gene": "UniProtKB:P49682",
  "term_label": "cell chemotaxis"
}